{
  "gene_symbol": "KCNK3",
  "term_id": "GO:0071805",
  "gene_name": "Potassium channel subfamily K member 3",
  "term_label": "potassium ion transmembrane transport",
  "gene": "UniProtKB:O14649"
}